histone locus body [GO:0035363] (cellular component) Definition: A nuclear body associated with the histone gene locus that is thought to contain all of the factors necessary for histone mRNA transcription and pre-mRNA processing. In Drosophila, U7 snRNP is located in the histone locus body rather than the distinct Cajal body. References: PMID:16533947, PMID:18927579, PMID:19620235 Sources: GOC:sart Also known as: HLB Relationships: is a type of nuclear ribonucleoprotein granule [GO:0140168]